{
  "gene_symbol": "SLC7A5",
  "term_id": "GO:0015175",
  "gene": "UniProtKB:Q01650",
  "gene_name": "Large neutral amino acids transporter small subunit 1",
  "term_label": "neutral L-amino acid transmembrane transporter activity"
}